{
  "gene_symbol": "FZD8",
  "term_label": "plasma membrane",
  "gene_name": "Frizzled-8",
  "term_id": "GO:0005886",
  "gene": "UniProtKB:Q9H461"
}